proteasome complex disassembly [GO:1903009] (biological process) Also known as: proteasome degradation, proteasome disassembly, 26S proteasome disassembly Definition: The disaggregation of a proteasome complex into its constituent components. Sources: GOC:TermGenie, GO_REF:0000079 Relationships: is a type of protein-containing complex disassembly [GO:0032984]